{
  "gene_symbol": "MTO1",
  "term_id": "GO:0050660",
  "term_label": "flavin adenine dinucleotide binding",
  "gene_name": "Protein MTO1 homolog, mitochondrial",
  "gene": "UniProtKB:Q9Y2Z2"
}